{
  "gene_name": "Small integral membrane protein 6",
  "term_id": "UNKNOWN:0001",
  "term_label": "Unknown molecular function",
  "gene_symbol": "SMIM6",
  "gene": "UniProtKB:P0DI80"
}